positive regulation of post-embryonic development [GO:0048582] (biological process) Subtypes: positive regulation of flower development [GO:0009911], positive regulation of seed germination [GO:0010030], GO:0048576, positive regulation of long-day photoperiodism, flowering [GO:0048578], positive regulation of nematode larval development [GO:0061063], positive regulation of thermomorphogenesis [GO:0140922], positive regulation of lateral root development [GO:1901333], positive regulation of stomatal complex development [GO:2000123], positive regulation of photomorphogenesis [GO:2000306] Sources: GOC:jid Also known as: up regulation of post-embryonic development, up-regulation of post-embryonic development, upregulation of post-embryonic development, activation of post-embryonic development, stimulation of post-embryonic development Definition: Any process that activates or increases the frequency, rate or extent of post-embryonic development. Post-embryonic development is defined as the process whose specific outcome is the progression of the organism over time, from the completion of embryonic development to the mature structure. Relationships: is a type of regulation of post-embryonic development [GO:0048580]; is a type of positive regulation of developmental process [GO:0051094]; is a type of positive regulation of multicellular organismal process [GO:0051240]; positively regulates post-embryonic development [GO:0009791]